post-lysosomal vacuole [GO:0032195] (cellular component) Definition: A membrane-bounded intracellular vesicle formed late in the endocytic pathway when the pH in the vacuole becomes neutral prior to exocytosis. References: PMID:23494323, PMID:9276759, PMID:9394012 Sources: GOC:pf Also known as: post-lysosome, postlysosome Relationships: is a type of vacuole [GO:0005773]; is a type of endocytic vesicle [GO:0030139]